{
  "gene_name": "Protein transport protein Sec61 subunit alpha isoform 1",
  "gene_symbol": "SEC61A1",
  "gene": "UniProtKB:P61619",
  "term_label": "Sec61 translocon complex",
  "term_id": "GO:0005784"
}